{
  "gene_name": "Teashirt homolog 1",
  "term_label": "DNA binding",
  "term_id": "GO:0003677",
  "gene": "UniProtKB:Q6ZSZ6",
  "gene_symbol": "TSHZ1"
}